calcium-dependent phospholipid binding [GO:0005544] (molecular function) Sources: GOC:jl Relationships: is a type of GO:0005543 Definition: Binding to a phospholipid, a class of lipids containing phosphoric acid as a mono- or diester, in the presence of calcium.